{
  "term_id": "GO:0071208",
  "gene_symbol": "LSM10",
  "gene": "UniProtKB:Q969L4",
  "gene_name": "U7 snRNA-associated Sm-like protein LSm10",
  "term_label": "histone pre-mRNA DCP binding"
}